tropinone reductase activity [GO:0050358] (molecular function) Definition: Catalysis of the reaction: NADP+ + pseudotropine = H+ + NADPH + tropinone. Sources: EC:1.1.1.236, RHEA:24244 Also known as: pseudotropine forming tropinone reductase activity, pseudotropine:NADP+ 3-oxidoreductase activity, tropinone (psi-tropine-forming) reductase activity, tropinone reductase II activity Relationships: is a type of GO:0016616